{
  "gene_symbol": "SLC9A3",
  "gene_name": "Sodium_hydrogen exchanger 3",
  "term_label": "sodium ion import across plasma membrane",
  "term_id": "GO:0098719",
  "gene": "UniProtKB:P48764"
}